{
  "gene": "UniProtKB:O14503",
  "gene_symbol": "BHLHE40",
  "term_label": "DNA-binding transcription factor activity, RNA polymerase II-specific",
  "gene_name": "Class E basic helix-loop-helix protein 40",
  "term_id": "GO:0000981"
}